{
  "term_id": "GO:0008250",
  "term_label": "oligosaccharyltransferase complex",
  "gene_name": "Tumor suppressor candidate 3",
  "gene_symbol": "TUSC3",
  "gene": "UniProtKB:Q13454"
}